{
  "term_id": "UNKNOWN:0001",
  "gene_name": "Uncharacterized protein C10orf55",
  "term_label": "Unknown molecular function",
  "gene": "UniProtKB:Q5SWW7",
  "gene_symbol": "C10orf55"
}